{
  "gene": "UniProtKB:P01718",
  "term_label": "immune response",
  "gene_symbol": "IGLV3-27",
  "term_id": "GO:0006955",
  "gene_name": "Immunoglobulin lambda variable 3-27"
}